{
  "gene_name": "Metallothionein 1H-like protein 1",
  "gene_symbol": "MT1HL1",
  "gene": "UniProtKB:P0DM35",
  "term_id": "GO:0005634",
  "term_label": "nucleus"
}